phosphatidic acid transfer activity [GO:1990050] (molecular function) Relationships: is a type of phospholipid transfer activity [GO:0120014] Definition: Removes a phosphatidic acid from a membrane or a monolayer lipid particle, transports it through the aqueous phase while protected in a hydrophobic pocket, and brings it to an acceptor membrane or lipid particle. Phosphatidic acid refers to a glycophospholipids with, in general, a saturated fatty acid bonded to carbon-1, an unsaturated fatty acid bonded to carbon-2, and a phosphate group bonded to carbon-3. References: PMID:23042293 Also known as: phosphatidic acid transporter activity, intermembrane PA transfer activity, phosphatidic acid carrier activity, intermembrane phosphatidic acid transfer activity